{
  "term_id": "GO:0005886",
  "gene_symbol": "SLA",
  "term_label": "plasma membrane",
  "gene": "UniProtKB:Q13239",
  "gene_name": "Src-like-adapter"
}